regulation of apoptotic DNA fragmentation [GO:1902510] (BP) Note: DNA fragmentation in response to apoptotic signals is achieved through the activity of apoptotic nucleases (see GO:0006309 'apoptotic DNA fragmentation'). Gene products involved in compartmentalization of such nucleases and in activation or repression of their enzymatic activity should be annotated to the regulation term GO:1902510 'regulation of apoptotic DNA fragmentation' or to one of its children (see PMID:15723341). References: PMID:15572351, PMID:15723341 Sources: GOC:TermGenie, GOC:hjd Definition: Any process that modulates the frequency, rate or extent of apoptotic DNA fragmentation. Also known as: regulation of DNA fragmentation, regulation of chromatinolysis, regulation of DNA catabolic process during apoptosis, regulation of DNA catabolism during apoptosis, regulation of DNA fragmentation involved in apoptotic nuclear change, regulation of endonucleolytic DNA catabolic process involved in apoptosis Subtypes: negative regulation of apoptotic DNA fragmentation [GO:1902511], positive regulation of apoptotic DNA fragmentation [GO:1902512] Relationships: is a type of GO:1903624; regulates apoptotic DNA fragmentation [GO:0006309]